regulation of odontoblast differentiation [GO:1901329] (biological process) Subtypes: negative regulation of odontoblast differentiation [GO:1901330], positive regulation of odontoblast differentiation [GO:1901331] Relationships: is a type of regulation of epithelial cell differentiation [GO:0030856]; regulates GO:0071895 Sources: GOC:TermGenie Definition: Any process that modulates the frequency, rate or extent of odontoblast differentiation.